{
  "term_label": "transcription factor TFIID complex",
  "term_id": "GO:0005669",
  "gene_name": "TATA-box-binding protein-associated factor 11-like protein 8",
  "gene_symbol": "TAF11L8",
  "gene": "UniProtKB:P0DW13"
}